{
  "gene": "UniProtKB:O00329",
  "term_id": "GO:0035005",
  "gene_name": "Phosphatidylinositol 4,5-bisphosphate 3-kinase catalytic subunit delta isoform",
  "term_label": "1-phosphatidylinositol-4-phosphate 3-kinase activity",
  "gene_symbol": "PIK3CD"
}